{
  "term_id": "GO:0005143",
  "gene_name": "Interleukin-12 subunit beta",
  "term_label": "interleukin-12 receptor binding",
  "gene": "UniProtKB:P29460",
  "gene_symbol": "IL12B"
}